{
  "gene": "UniProtKB:Q96QU6",
  "gene_name": "1-aminocyclopropane-1-carboxylate synthase-like protein 1",
  "term_label": "transaminase activity",
  "term_id": "GO:0008483",
  "gene_symbol": "ACCS"
}